{
  "term_label": "negative regulation of ERAD pathway",
  "gene": "UniProtKB:Q8NHG7",
  "gene_symbol": "SVIP",
  "term_id": "GO:1904293",
  "gene_name": "Small VCP_p97-interacting protein"
}